{
  "gene_symbol": "ZNF557",
  "gene": "UniProtKB:Q8N988",
  "term_label": "regulation of transcription by RNA polymerase II",
  "term_id": "GO:0006357",
  "gene_name": "Zinc finger protein 557"
}